{
  "gene_name": "Actin, cytoplasmic 1",
  "term_label": "axonogenesis",
  "gene_symbol": "ACTB",
  "gene": "UniProtKB:P60709",
  "term_id": "GO:0007409"
}